{
  "gene_name": "Neuromedin-U receptor 2",
  "term_id": "GO:0007200",
  "gene_symbol": "NMUR2",
  "term_label": "phospholipase C-activating G protein-coupled receptor signaling pathway",
  "gene": "UniProtKB:Q9GZQ4"
}